{
  "gene_symbol": "ACER3",
  "gene": "UniProtKB:Q9NUN7",
  "term_label": "phytosphingosine biosynthetic process",
  "term_id": "GO:0071602",
  "gene_name": "Alkaline ceramidase 3"
}